{
  "gene": "UniProtKB:Q5DX21",
  "gene_name": "Immunoglobulin superfamily member 11",
  "term_label": "Unknown molecular function",
  "gene_symbol": "IGSF11",
  "term_id": "UNKNOWN:0001"
}